{
  "term_label": "Unknown molecular function",
  "gene_symbol": "DRICH1",
  "gene": "UniProtKB:Q6PGQ1",
  "gene_name": "Aspartate-rich protein 1",
  "term_id": "UNKNOWN:0001"
}